{
  "gene": "UniProtKB:Q8N1T3",
  "term_id": "GO:0005902",
  "term_label": "microvillus",
  "gene_name": "Unconventional myosin-Ih",
  "gene_symbol": "MYO1H"
}